{
  "gene_symbol": "CPLX1",
  "term_id": "GO:0031630",
  "gene": "UniProtKB:O14810",
  "term_label": "regulation of synaptic vesicle fusion to presynaptic active zone membrane",
  "gene_name": "Complexin-1"
}